{
  "term_id": "GO:1902093",
  "gene_symbol": "TACR2",
  "term_label": "positive regulation of flagellated sperm motility",
  "gene_name": "Substance-K receptor",
  "gene": "UniProtKB:P21452"
}